negative regulation of dendritic cell differentiation [GO:2001199] (biological process) Relationships: is a type of negative regulation of leukocyte differentiation [GO:1902106]; is a type of regulation of dendritic cell differentiation [GO:2001198]; negatively regulates dendritic cell differentiation [GO:0097028] Sources: GOC:obol Definition: Any process that stops, prevents or reduces the frequency, rate or extent of dendritic cell differentiation.